{
  "gene_symbol": "BMPR1A",
  "gene_name": "Bone morphogenetic protein receptor type-1A",
  "gene": "UniProtKB:P36894",
  "term_id": "GO:0071363",
  "term_label": "cellular response to growth factor stimulus"
}